{
  "term_id": "GO:0000776",
  "term_label": "kinetochore",
  "gene": "UniProtKB:P0DPK5",
  "gene_name": "Histone H3.X",
  "gene_symbol": "H3Y2"
}